{
  "gene_symbol": "KNTC1",
  "gene_name": "Kinetochore-associated protein 1",
  "gene": "UniProtKB:P50748",
  "term_label": "kinetochore microtubule",
  "term_id": "GO:0005828"
}